C-palmitoyltransferase activity [GO:0016454] (molecular function) Subtypes: serine C-palmitoyltransferase activity [GO:0004758] Definition: Catalysis of the transfer of a palmitoyl group to a carbon atom on the acceptor molecule. Sources: GOC:ai Relationships: is a type of C-acyltransferase activity [GO:0016408]; is a type of palmitoyltransferase activity [GO:0016409]